{
  "term_label": "protein kinase binding",
  "gene_name": "Protein FAM83G",
  "gene": "UniProtKB:A6ND36",
  "gene_symbol": "FAM83G",
  "term_id": "GO:0019901"
}